{
  "gene": "UniProtKB:Q15648",
  "gene_symbol": "MED1",
  "gene_name": "Mediator of RNA polymerase II transcription subunit 1",
  "term_id": "GO:0042809",
  "term_label": "nuclear vitamin D receptor binding"
}